skeletal muscle acetylcholine-gated channel clustering [GO:0071340] (biological process) References: PMID:19285469 Sources: GOC:bf, GOC:dsf Definition: The accumulation of acetylcholine-gated cation channels in a narrow, central region of muscle fibers, in apposition to nerve terminals. Also known as: skeletal muscle AChR clustering, skeletal muscle nicotinic acetylcholine receptor clustering Regulation: regulated by regulation of skeletal muscle acetylcholine-gated channel clustering [GO:1904393]; negatively regulated by negative regulation of skeletal muscle acetylcholine-gated channel clustering [GO:1904394]; positively regulated by GO:1904395 Relationships: is a type of receptor clustering [GO:0043113]; is part of postsynaptic membrane organization [GO:0001941]; is part of GO:0007528